female germ-line stem cell population maintenance [GO:0036099] (biological process) Definition: The process by which an organism or tissue maintains a population of female germ-line stem cells. Relationships: is a type of GO:0030718 Sources: GOC:sart